monoatomic ion channel complex [GO:0034702] (cellular component) Sources: GOC:mah, ISBN:071673706X Definition: A protein complex that spans a membrane and forms a water-filled channel across the phospholipid bilayer allowing selective monoatomic ion transport down its electrochemical gradient. Relationships: is_a transmembrane transporter complex [GO:1902495] Subtypes: acetylcholine-gated channel complex [GO:0005892], ionotropic glutamate receptor complex [GO:0008328], cation channel complex [GO:0034703], chloride channel complex [GO:0034707]